guanylate kinase-associated protein clustering [GO:0097117] (biological process) Definition: The clustering process in which guanylate kinase-associated proteins (GKAPs) are localized to distinct domains in the cell membrane. GKAP facilitates assembly of the post synaptic density of neurons. Also known as: GKAP clustering Relationships: is a type of GO:0072657; is part of postsynaptic membrane organization [GO:0001941] References: PMID:15620359 Sources: GOC:BHF, GOC:sjp